3-hydroxyphenylacetate 6-hydroxylase activity [GO:0047094] (MF) Definition: Catalysis of the reaction: O2 + NAD(P)H + 3-hydroxyphenylacetate = H2O + NAD(P)+ + homogentisate. Relationships: is a type of GO:0016709 Sources: EC:1.14.13.63 Also known as: 3-hydroxyphenylacetate 6-monooxygenase activity, 3-hydroxyphenylacetate,NAD(P)H:oxygen oxidoreductase (6-hydroxylating)